{
  "term_id": "GO:0046875",
  "gene": "UniProtKB:O43921",
  "gene_name": "Ephrin-A2",
  "term_label": "ephrin receptor binding",
  "gene_symbol": "EFNA2"
}